{
  "gene": "UniProtKB:Q96QK8",
  "term_id": "UNKNOWN:0002",
  "gene_name": "Small integral membrane protein 14",
  "term_label": "Unknown biological process",
  "gene_symbol": "SMIM14"
}